{
  "gene": "UniProtKB:P09564",
  "gene_symbol": "CD7",
  "term_id": "UNKNOWN:0002",
  "term_label": "Unknown biological process",
  "gene_name": "T-cell antigen CD7"
}